{
  "term_id": "UNKNOWN:0002",
  "gene": "UniProtKB:Q6L8H2",
  "gene_name": "Keratin-associated protein 5-3",
  "gene_symbol": "KRTAP5-3",
  "term_label": "Unknown biological process"
}